{
  "term_label": "negative regulation of inflammatory response",
  "gene_symbol": "OTULIN",
  "gene_name": "Ubiquitin thioesterase otulin",
  "gene": "UniProtKB:Q96BN8",
  "term_id": "GO:0050728"
}